{
  "gene_name": "Beta-secretase 1",
  "term_label": "plasma membrane",
  "term_id": "GO:0005886",
  "gene_symbol": "BACE1",
  "gene": "UniProtKB:P56817"
}